{
  "gene": "UniProtKB:Q9BXL5",
  "gene_name": "Hemogen",
  "term_label": "Unknown molecular function",
  "term_id": "UNKNOWN:0001",
  "gene_symbol": "HEMGN"
}